{
  "gene_name": "C5a anaphylatoxin chemotactic receptor 2",
  "term_label": "complement component C5a receptor activity",
  "term_id": "GO:0004878",
  "gene_symbol": "C5AR2",
  "gene": "UniProtKB:Q9P296"
}